{
  "term_label": "nucleolus",
  "gene": "UniProtKB:Q9NVU7",
  "gene_name": "Protein SDA1 homolog",
  "gene_symbol": "SDAD1",
  "term_id": "GO:0005730"
}